{
  "gene_name": "Protein ERGIC-53",
  "gene": "UniProtKB:P49257",
  "term_label": "COPII-coated ER to Golgi transport vesicle",
  "term_id": "GO:0030134",
  "gene_symbol": "LMAN1"
}